{
  "term_label": "kinase binding",
  "term_id": "GO:0019900",
  "gene": "UniProtKB:Q9H6R7",
  "gene_symbol": "WDCP",
  "gene_name": "WD repeat and coiled-coil-containing protein"
}